dTDP catabolic process [GO:0006246] (biological process) Relationships: is a type of GO:0009198; is a type of GO:0009223; is a type of GO:0046072 Definition: The chemical reactions and pathways resulting in the breakdown of dTDP, deoxyribosylthymine diphosphate. Also known as: dTDP breakdown, dTDP catabolism, dTDP degradation Sources: ISBN:0198506732